{
  "gene_symbol": "CPNE9",
  "term_label": "plasma membrane",
  "gene": "UniProtKB:Q8IYJ1",
  "gene_name": "Copine-9",
  "term_id": "GO:0005886"
}